{
  "term_label": "sarcomere organization",
  "gene_symbol": "MYBPH",
  "gene": "UniProtKB:Q13203",
  "term_id": "GO:0045214",
  "gene_name": "Myosin-binding protein H"
}